{
  "gene_name": "Gamma-secretase subunit APH-1B",
  "term_label": "Notch receptor processing",
  "gene": "UniProtKB:Q8WW43",
  "gene_symbol": "APH1B",
  "term_id": "GO:0007220"
}